{
  "term_label": "receptor ligand activity",
  "gene": "UniProtKB:Q96LR4",
  "gene_symbol": "TAFA4",
  "term_id": "GO:0048018",
  "gene_name": "Chemokine-like protein TAFA-4"
}